regulation of membrane disassembly [GO:0010549] (biological process) Subtypes: regulation of thylakoid membrane disassembly [GO:0010548], regulation of mitotic nuclear envelope disassembly [GO:1905557] Sources: GOC:dph, GOC:tb Definition: Any process that modulates the frequency, rate or extent of membrane disassembly. Relationships: is a type of regulation of cellular component organization [GO:0051128]; regulates membrane disassembly [GO:0030397]